negative regulation of synaptic transmission, cholinergic [GO:0032223] (biological process) Sources: GOC:mah Definition: Any process that stops, prevents, or reduces the frequency, rate or extent of cholinergic synaptic transmission, the process of communication from a neuron to another neuron across a synapse using the neurotransmitter acetylcholine. Also known as: down regulation of synaptic transmission, cholinergic, down-regulation of synaptic transmission, cholinergic, downregulation of synaptic transmission, cholinergic, inhibition of synaptic transmission, cholinergic Subtypes: GO:0014058 Relationships: is a type of regulation of synaptic transmission, cholinergic [GO:0032222]; is a type of GO:0050805; negatively regulates synaptic transmission, cholinergic [GO:0007271]